mitotic chromosome arm condensation [GO:1990892] (biological process) References: PMID:21633354 Relationships: is a type of mitotic chromosome condensation [GO:0007076] Definition: The cell cycle process in which chromosome arm chromatin structure is compacted prior to and during mitosis in eukaryotic cells.